{
  "gene": "UniProtKB:O95998",
  "gene_symbol": "IL18BP",
  "gene_name": "Interleukin-18-binding protein",
  "term_id": "GO:0042088",
  "term_label": "T-helper 1 type immune response"
}